{
  "term_label": "Unknown biological process",
  "gene_name": "Inter-alpha-trypsin inhibitor heavy chain H6",
  "gene": "UniProtKB:Q6UXX5",
  "gene_symbol": "ITIH6",
  "term_id": "UNKNOWN:0002"
}